{
  "term_label": "mitochondrion",
  "gene_name": "Mitochondrial ornithine transporter 2",
  "term_id": "GO:0005739",
  "gene": "UniProtKB:Q9BXI2",
  "gene_symbol": "SLC25A2"
}